positive regulation of fractalkine production [GO:0032724] (biological process) Sources: GOC:mah Definition: Any process that activates or increases the frequency, rate, or extent of fractalkine production. Relationships: is_a regulation of fractalkine production [GO:0032644]; is a type of GO:0032722; positively regulates fractalkine production [GO:0032603] Also known as: up regulation of fractalkine production, up-regulation of fractalkine production, upregulation of fractalkine production, activation of fractalkine production, stimulation of fractalkine production